UDP-D-xylose biosynthetic process [GO:0033320] (biological process) Definition: The chemical reactions and pathways resulting in the formation of UDP-D-xylose, uridinediphosphoxylose, a substance composed of xylose in glycosidic linkage with uridine diphosphate. Sources: GOC:mah, MetaCyc:PWY-4821 Also known as: UDP-D-xylose anabolism, UDP-D-xylose biosynthesis, UDP-D-xylose formation, UDP-D-xylose synthesis Relationships: is a type of GO:0009226; is a type of UDP-D-xylose metabolic process [GO:0033319]